commissural neuron differentiation in spinal cord [GO:0021528] (biological process) References: PMID:11262869 Sources: GOC:cls, GOC:dgh, GOC:dph, GOC:jid, GO_REF:0000021 Relationships: is a type of GO:0021515; is a type of GO:0021953 Definition: The process in which neuroepithelial cells in the ventral neural tube acquire specialized structural and/or functional features of commissural neurons. Commissural neurons in both vertebrates and invertebrates transfer information from one side of their bodies to the other through the midline. Differentiation includes the processes involved in commitment of a cell to a specific fate.